{
  "term_id": "UNKNOWN:0001",
  "term_label": "Unknown molecular function",
  "gene_symbol": "INO80C",
  "gene": "UniProtKB:Q6PI98",
  "gene_name": "INO80 complex subunit C"
}